{
  "gene_symbol": "GATA6",
  "gene_name": "Transcription factor GATA-6",
  "term_label": "negative regulation of transcription by RNA polymerase II",
  "term_id": "GO:0000122",
  "gene": "UniProtKB:Q92908"
}